{
  "gene_name": "AP-4 complex accessory subunit RUSC1",
  "term_id": "UNKNOWN:0002",
  "gene_symbol": "RUSC1",
  "gene": "UniProtKB:Q9BVN2",
  "term_label": "Unknown biological process"
}